{
  "gene_symbol": "TMEM33",
  "term_id": "UNKNOWN:0001",
  "term_label": "Unknown molecular function",
  "gene": "UniProtKB:P57088",
  "gene_name": "Transmembrane protein 33"
}